{
  "term_label": "SCF-dependent proteasomal ubiquitin-dependent protein catabolic process",
  "term_id": "GO:0031146",
  "gene_name": "F-box_LRR-repeat protein 20",
  "gene": "UniProtKB:Q96IG2",
  "gene_symbol": "FBXL20"
}